{
  "gene": "UniProtKB:P52789",
  "gene_symbol": "HK2",
  "term_id": "GO:0006006",
  "term_label": "glucose metabolic process",
  "gene_name": "Hexokinase-2"
}